azetidine-2-carboxylic acid acetyltransferase activity [GO:0046941] (molecular function) References: PMID:12761200 Definition: Catalysis of the reaction: L-azetidine-2-carboxylic acid + acetyl-CoA = CoA-SH + N-acetyl azetidine-2-carboxylic acid. Relationships: is a type of N-acetyltransferase activity [GO:0008080]